{
  "gene": "UniProtKB:Q9H9L4",
  "gene_symbol": "KANSL2",
  "gene_name": "KAT8 regulatory NSL complex subunit 2",
  "term_id": "UNKNOWN:0002",
  "term_label": "Unknown biological process"
}